{
  "gene_symbol": "CELSR3",
  "term_label": "plasma membrane",
  "gene_name": "Cadherin EGF LAG seven-pass G-type receptor 3",
  "term_id": "GO:0005886",
  "gene": "UniProtKB:Q9NYQ7"
}